{
  "gene": "UniProtKB:Q2QD12",
  "term_id": "GO:0005975",
  "gene_name": "Ribulose-phosphate 3-epimerase-like protein 1",
  "gene_symbol": "RPEL1",
  "term_label": "carbohydrate metabolic process"
}